regulation of membrane lipid distribution [GO:0097035] (biological process) Relationships: is a type of membrane organization [GO:0061024]; is a type of regulation of biological quality [GO:0065008] Definition: Any process that modulates the proportions or spatial arrangement of lipids in a cellular membrane. References: PMID:18441123, PMID:20823909 Sources: GOC:mah Subtypes: lipid translocation [GO:0034204], regulation of phospholipid translocation [GO:0061091], regulation of plasma membrane sterol distribution [GO:0097036]